response to amphetamine [GO:0001975] (biological process) Definition: Any process that results in a change in state or activity of a cell or an organism (in terms of movement, secretion, enzyme production, gene expression, etc.) as a result of an amphetamine stimulus. Amphetamines consist of a group of compounds related to alpha-methylphenethylamine. Sources: GOC:dph, GOC:ef Relationships: is a type of GO:0014075 Subtypes: cellular response to amphetamine [GO:0071419]